regulation of DNA damage checkpoint [GO:2000001] (biological process) Sources: GOC:obol Subtypes: regulation of mitotic DNA damage checkpoint [GO:1904289], negative regulation of DNA damage checkpoint [GO:2000002], GO:2000003 Definition: Any process that modulates the frequency, rate or extent of a DNA damage checkpoint. Relationships: is a type of GO:0080135; is a type of GO:1901976; regulates DNA damage checkpoint signaling [GO:0000077] Also known as: regulation of DNA damage response, signal transduction resulting in cell cycle arrest